{
  "term_label": "Unknown molecular function",
  "gene": "UniProtKB:P98153",
  "gene_name": "Integral membrane protein DGCR2_IDD",
  "term_id": "UNKNOWN:0001",
  "gene_symbol": "DGCR2"
}